dense core granule organization [GO:0061109] (biological process) Definition: A process that is carried out at the cellular level which results in the assembly, arrangement of constituent parts, or disassembly of a dense core granule. A dense core granule is a secretory organelle found in endocrine cells. Sources: GOC:dph Also known as: dense core granule organisation Relationships: is a type of secretory granule organization [GO:0033363] Subtypes: neuronal dense core vesicle organization [GO:0099014]